positive regulation of connective tissue replacement [GO:1905205] (biological process) Relationships: is a type of positive regulation of tissue remodeling [GO:0034105]; is a type of GO:1905203; positively regulates connective tissue replacement [GO:0097709] Also known as: up regulation of connective tissue replacement, up-regulation of connective tissue replacement, upregulation of connective tissue replacement, activation of connective tissue replacement References: PMID:25590961 Sources: GOC:BHF, GOC:BHF_miRNA, GOC:TermGenie, GOC:bc, GO_REF:0000058 Subtypes: positive regulation of connective tissue replacement involved in inflammatory response wound healing [GO:1904598] Definition: Any process that activates or increases the frequency, rate or extent of connective tissue replacement.